{
  "gene_symbol": "ENKD1",
  "gene_name": "Enkurin domain-containing protein 1",
  "gene": "UniProtKB:Q9H0I2",
  "term_label": "cytoplasmic microtubule",
  "term_id": "GO:0005881"
}